{
  "term_id": "GO:0000981",
  "term_label": "DNA-binding transcription factor activity, RNA polymerase II-specific",
  "gene_symbol": "ZNF492",
  "gene": "UniProtKB:Q9P255",
  "gene_name": "Zinc finger protein 492"
}